fumarylpyruvate hydrolase activity [GO:0034545] (molecular function) Definition: Catalysis of the reaction: fumarylpyruvate + H2O = fumarate + pyruvate + H+. Sources: UM-BBD_reactionID:r0811 Relationships: is a type of hydrolase activity, acting on acid carbon-carbon bonds, in ketonic substances [GO:0016823]